{
  "term_id": "UNKNOWN:0001",
  "gene": "UniProtKB:Q9H6D3",
  "gene_symbol": "XKR8",
  "term_label": "Unknown molecular function",
  "gene_name": "XK-related protein 8"
}